{
  "gene_symbol": "SLC30A4",
  "term_id": "GO:0005385",
  "gene": "UniProtKB:O14863",
  "term_label": "zinc ion transmembrane transporter activity",
  "gene_name": "Probable proton-coupled zinc antiporter SLC30A4"
}